{
  "term_id": "GO:0004497",
  "term_label": "monooxygenase activity",
  "gene": "UniProtKB:O43174",
  "gene_name": "Cytochrome P450 26A1",
  "gene_symbol": "CYP26A1"
}